{
  "gene": "UniProtKB:Q8IUQ0",
  "term_label": "clathrin-coated vesicle",
  "gene_symbol": "CLVS1",
  "gene_name": "Clavesin-1",
  "term_id": "GO:0030136"
}